FMN metabolic process [GO:0046444] (biological process) Definition: The chemical reactions and pathways involving FMN, riboflavin 5'-(dihydrogen phosphate), a coenzyme for a number of oxidative enzymes including NADH dehydrogenase. References: PMID:20822113 Sources: GOC:ai Also known as: FMN metabolism Relationships: is a type of nucleoside monophosphate metabolic process [GO:0009123]; is_a ribonucleotide metabolic process [GO:0009259]; is a type of flavin-containing compound metabolic process [GO:0042726] Subtypes: FMN biosynthetic process [GO:0009398], FMN catabolic process [GO:0032363]